{
  "gene": "UniProtKB:Q8NGS5",
  "gene_name": "Olfactory receptor 13C4",
  "gene_symbol": "OR13C4",
  "term_label": "plasma membrane",
  "term_id": "GO:0005886"
}